{
  "term_id": "GO:0007169",
  "term_label": "cell surface receptor protein tyrosine kinase signaling pathway",
  "gene_name": "Macrophage colony-stimulating factor 1 receptor",
  "gene_symbol": "CSF1R",
  "gene": "UniProtKB:P07333"
}